{
  "term_id": "GO:0005576",
  "gene": "UniProtKB:Q8NAU1",
  "gene_name": "Fibronectin type III domain-containing protein 5",
  "gene_symbol": "FNDC5",
  "term_label": "extracellular region"
}